{
  "term_label": "plasma membrane",
  "term_id": "GO:0005886",
  "gene": "UniProtKB:Q9HCU4",
  "gene_symbol": "CELSR2",
  "gene_name": "Cadherin EGF LAG seven-pass G-type receptor 2"
}